mitochondrion distribution [GO:0048311] (biological process) Definition: Any process that establishes the spatial arrangement of mitochondria between and within cells. Subtypes: mitochondrion inheritance [GO:0000001], GO:0048312, mitocytosis [GO:0160040] Sources: GOC:jid Also known as: distribution of mitochondria, mitochondrial distribution, positioning of mitochondria Relationships: is a type of GO:0051646